{
  "gene_symbol": "GPR132",
  "term_label": "negative regulation of G2/M transition of mitotic cell cycle",
  "gene": "UniProtKB:Q9UNW8",
  "term_id": "GO:0010972",
  "gene_name": "Probable G-protein coupled receptor 132"
}